abscisic acid glucosyltransferase activity [GO:0010294] (molecular function) Definition: Catalysis of the reaction: (+)-abscisate + UDP-D-glucose = abscisic acid glucose ester + UDP. Sources: DOI:10.1016/j.tetasy.2004.11.062 Relationships: is a type of GO:0035251